{
  "term_label": "histone binding",
  "gene_symbol": "WDR5",
  "gene": "UniProtKB:P61964",
  "gene_name": "WD repeat-containing protein 5",
  "term_id": "GO:0042393"
}